{
  "term_id": "GO:0016064",
  "term_label": "immunoglobulin mediated immune response",
  "gene_symbol": "IGHV3OR16-13",
  "gene_name": "Immunoglobulin heavy variable 3_OR16-13 (non-functional) (Fragment)",
  "gene": "UniProtKB:A0A075B7E8"
}